{
  "term_id": "GO:0005737",
  "term_label": "cytoplasm",
  "gene_name": "Peptidyl-prolyl cis-trans isomerase H",
  "gene_symbol": "PPIH",
  "gene": "UniProtKB:O43447"
}